positive regulation of salivary gland boundary specification [GO:0045706] (biological process) Also known as: positive regulation of salivary gland determination, up regulation of salivary gland determination, up-regulation of salivary gland determination, upregulation of salivary gland determination, activation of salivary gland determination, stimulation of salivary gland determination Definition: Any process that activates or increases the frequency, rate or extent of salivary gland determination. Subtypes: positive regulation of adult salivary gland boundary specification [GO:0045711], positive regulation of larval salivary gland boundary specification [GO:0045712] Sources: GOC:go_curators, GOC:tb Relationships: is a type of regulation of salivary gland boundary specification [GO:0045704]; is a type of positive regulation of developmental process [GO:0051094]; is a type of positive regulation of multicellular organismal process [GO:0051240]; positively regulates salivary gland boundary specification [GO:0007432]